negative regulation of acute inflammatory response to non-antigenic stimulus [GO:0002878] (biological process) Definition: Any process that stops, prevents, or reduces the frequency, rate, or extent of an acute inflammatory response to a non-antigenic stimulus. Also known as: down regulation of acute inflammatory response to non-antigenic stimulus, down-regulation of acute inflammatory response to non-antigenic stimulus, downregulation of acute inflammatory response to non-antigenic stimulus, inhibition of acute inflammatory response to non-antigenic stimulus Sources: GOC:add Relationships: is a type of negative regulation of acute inflammatory response [GO:0002674]; is a type of GO:0002877; negatively regulates acute inflammatory response to non-antigenic stimulus [GO:0002525]